{
  "term_label": "Unknown biological process",
  "term_id": "UNKNOWN:0002",
  "gene_symbol": "FAM223A",
  "gene_name": "Protein FAM223A",
  "gene": "UniProtKB:Q8IWN6"
}